{
  "term_id": "UNKNOWN:0003",
  "gene": "UniProtKB:P23760",
  "gene_symbol": "PAX3",
  "term_label": "Unknown cellular component",
  "gene_name": "Paired box protein Pax-3"
}